{
  "gene": "UniProtKB:Q13888",
  "gene_symbol": "GTF2H2",
  "term_id": "UNKNOWN:0001",
  "term_label": "Unknown molecular function",
  "gene_name": "General transcription factor IIH subunit 2"
}